somatostatin receptor binding [GO:0031877] (molecular function) Subtypes: GO:0031878, GO:0031879, type 3 somatostatin receptor binding [GO:0031880], type 4 somatostatin receptor binding [GO:0031881], type 5 somatostatin receptor binding [GO:0031882] Also known as: somatostatin receptor ligand Relationships: is a type of GO:0071855 Definition: Binding to a somatostatin receptor. Sources: GOC:mah, GOC:nln